{
  "gene_symbol": "MAP1LC3A",
  "gene": "UniProtKB:Q9H492",
  "term_label": "microtubule binding",
  "gene_name": "Microtubule-associated proteins 1A_1B light chain 3A",
  "term_id": "GO:0008017"
}